chorion-containing eggshell pattern formation [GO:0030381] (biological process) Relationships: is a type of regionalization [GO:0003002]; is a type of GO:0003006; is part of chorion-containing eggshell formation [GO:0007304] Sources: GOC:bf, GOC:mtg_sensu Definition: The regionalization process that gives rise to the structural pattern of a chorion-containing eggshell such as those found in insects.